{
  "gene_name": "Suppressor of tumorigenicity 7 protein",
  "gene": "UniProtKB:Q9NRC1",
  "term_label": "Unknown biological process",
  "gene_symbol": "ST7",
  "term_id": "UNKNOWN:0002"
}